{
  "gene_symbol": "PNLIPRP2",
  "term_label": "extracellular space",
  "gene": "UniProtKB:P54317",
  "term_id": "GO:0005615",
  "gene_name": "Pancreatic lipase-related protein 2"
}